beta-catenin-ICAT complex [GO:1990711] (cellular component) Note: An example of this is Catenin beta-1 in human (UniProt symbol P35222) in PMID:12408824 (inferred from physical interaction). Relationships: is a type of RNA polymerase II transcription repressor complex [GO:0090571] References: PMID:12408824 Sources: GOC:bhm Also known as: CTNNB1-CTNNBIP1 complex Definition: Transcription factor complex that inhibits binding of Tcf to beta-catenin while preserving interaction of catenin with cadherin thus inhibiting transcription mediated by beta-catenin-Tcf complex.